{
  "term_id": "GO:0005005",
  "term_label": "transmembrane-ephrin receptor activity",
  "gene_symbol": "EPHA7",
  "gene_name": "Ephrin type-A receptor 7",
  "gene": "UniProtKB:Q15375"
}